presynaptic signal transduction [GO:0098928] (biological process) Definition: Signal transduction in which the initial step occurs in a presynapse. Sources: GOC:dos Also known as: presynaptic signaling pathway Relationships: is_a signal transduction [GO:0007165] Subtypes: presynapse to nucleus signaling pathway [GO:0099526]